{
  "gene_name": "Uncharacterized protein C16orf46",
  "gene": "UniProtKB:Q6P387",
  "term_label": "Unknown cellular component",
  "term_id": "UNKNOWN:0003",
  "gene_symbol": "C16orf46"
}